{
  "gene_name": "Keratin-associated protein 12-4",
  "term_label": "Unknown molecular function",
  "term_id": "UNKNOWN:0001",
  "gene": "UniProtKB:P60329",
  "gene_symbol": "KRTAP12-4"
}